{
  "gene_name": "NKG2-D type II integral membrane protein",
  "term_label": "external side of plasma membrane",
  "gene": "UniProtKB:P26718",
  "term_id": "GO:0009897",
  "gene_symbol": "KLRK1"
}